regulation of tissue kallikrein-kinin cascade [GO:0002382] (biological process) Sources: GOC:add Definition: Any process that modulates the frequency, rate, or extent of the tissue kallikrein-kinin cascade. Relationships: is a type of GO:0002256; regulates tissue kallikrein-kinin cascade [GO:0002255] Also known as: regulation of glandular kallikrein-kinin cascade Subtypes: negative regulation of tissue kallikrein-kinin cascade [GO:0002546], positive regulation of tissue kallikrein-kinin cascade [GO:0002547]